{
  "term_label": "SREBP signaling pathway",
  "gene_name": "Insulin-induced gene 1 protein",
  "gene_symbol": "INSIG1",
  "gene": "UniProtKB:O15503",
  "term_id": "GO:0032933"
}